{
  "term_label": "transcription coactivator activity",
  "gene_name": "Host cell factor 2",
  "gene": "UniProtKB:Q9Y5Z7",
  "gene_symbol": "HCFC2",
  "term_id": "GO:0003713"
}